negative regulation of glutamate secretion [GO:0014050] (biological process) Subtypes: negative regulation of glutamate secretion, neurotransmission [GO:1903295] Definition: Any process that stops, prevents, or reduces the frequency, rate or extent of the controlled release of glutamate. Relationships: is a type of regulation of glutamate secretion [GO:0014048]; is a type of negative regulation of organic acid transport [GO:0032891]; is a type of negative regulation of amino acid transport [GO:0051956]; is a type of negative regulation of secretion by cell [GO:1903531]; negatively regulates glutamate secretion [GO:0014047] Also known as: down regulation of glutamate secretion, down-regulation of glutamate secretion, downregulation of glutamate secretion, inhibition of glutamate secretion Sources: GOC:ef